{
  "gene": "UniProtKB:P52333",
  "term_id": "GO:0007259",
  "term_label": "cell surface receptor signaling pathway via JAK-STAT",
  "gene_name": "Tyrosine-protein kinase JAK3",
  "gene_symbol": "JAK3"
}